anterior rotation of the optic cup [GO:0003410] (biological process) Definition: A 90 degree-rotation of the optic cup resulting in its alignment with the anterior-posterior body axis. Sources: GOC:ascb_2009, GOC:dph, GOC:tb Relationships: is_a anatomical structure development [GO:0048856]; is part of camera-type eye development [GO:0043010]